{
  "gene_name": "Gremlin-1",
  "gene": "UniProtKB:O60565",
  "term_label": "sequestering of BMP from receptor via BMP binding",
  "gene_symbol": "GREM1",
  "term_id": "GO:0038098"
}